{
  "gene_symbol": "NEUROD6",
  "gene_name": "Neurogenic differentiation factor 6",
  "term_label": "axon development",
  "gene": "UniProtKB:Q96NK8",
  "term_id": "GO:0061564"
}